{
  "term_id": "GO:0004029",
  "gene": "UniProtKB:O94788",
  "gene_name": "Retinal dehydrogenase 2",
  "gene_symbol": "ALDH1A2",
  "term_label": "aldehyde dehydrogenase (NAD+) activity"
}